{
  "gene_name": "Disintegrin and metalloproteinase domain-containing protein 21",
  "term_id": "GO:1990913",
  "gene": "UniProtKB:Q9UKJ8",
  "gene_symbol": "ADAM21",
  "term_label": "sperm head plasma membrane"
}